glyceraldehyde-3-phosphate catabolic process [GO:0019683] (biological process) Relationships: is a type of glyceraldehyde-3-phosphate metabolic process [GO:0019682]; is a type of aldehyde catabolic process [GO:0046185]; is a type of organophosphate catabolic process [GO:0046434]; is a type of carbohydrate derivative catabolic process [GO:1901136] Also known as: glyceraldehyde 3-phosphate catabolic process, glyceraldehyde 3-phosphate catabolism, glyceraldehyde-3-phosphate breakdown, glyceraldehyde-3-phosphate catabolism, glyceraldehyde-3-phosphate degradation Definition: The chemical reactions and pathways resulting in the breakdown of glyceraldehyde-3-phosphate, an important intermediate in glycolysis. Sources: ISBN:0198506732